{
  "term_label": "cytosol",
  "gene_name": "6-phosphofructo-2-kinase_fructose-2,6-bisphosphatase 1",
  "term_id": "GO:0005829",
  "gene": "UniProtKB:P16118",
  "gene_symbol": "PFKFB1"
}